mesonephric juxtaglomerulus cell fate commitment [GO:0061230] (biological process) Sources: GOC:mtg_kidney_jan10 Definition: The process in which the developmental fate of a cell becomes restricted such that it will develop into a mesonephric juxtaglomerulus cell. Relationships: is a type of juxtaglomerulus cell fate commitment [GO:0072150]; is part of mesonephric juxtaglomerulus cell differentiation [GO:0061207]